{
  "term_id": "GO:0005737",
  "gene_name": "Dipeptidyl peptidase 3",
  "term_label": "cytoplasm",
  "gene_symbol": "DPP3",
  "gene": "UniProtKB:Q9NY33"
}